regulation of axial mesodermal cell fate determination [GO:0048324] (biological process) Sources: GOC:dgh Subtypes: GO:0048325, GO:0048326 Relationships: is a type of regulation of mesodermal cell fate determination [GO:0048334]; regulates GO:0048323 Definition: Any process that modulates the frequency, rate or extent of axial mesoderm cell fate determination.